{
  "gene_symbol": "SUPT7L",
  "gene_name": "STAGA complex 65 subunit gamma",
  "term_id": "GO:0003713",
  "term_label": "transcription coactivator activity",
  "gene": "UniProtKB:O94864"
}